{
  "term_id": "GO:0005654",
  "term_label": "nucleoplasm",
  "gene": "UniProtKB:Q9UBS0",
  "gene_symbol": "RPS6KB2",
  "gene_name": "Ribosomal protein S6 kinase beta-2"
}